{
  "gene_name": "Brain-specific serine protease 4",
  "gene_symbol": "PRSS22",
  "gene": "UniProtKB:Q9GZN4",
  "term_id": "GO:0008236",
  "term_label": "serine-type peptidase activity"
}